cardiac atrium formation [GO:0003210] (biological process) Definition: The developmental process pertaining to the initial formation of a cardiac atrium from unspecified parts. A cardiac atrium receives blood from a vein and pumps it to a cardiac ventricle. Subtypes: GO:0003216, cardiac right atrium formation [GO:0003217] Sources: GOC:mtg_heart Relationships: is a type of cardiac chamber formation [GO:0003207]; is part of cardiac atrium morphogenesis [GO:0003209]